cytochrome c biosynthetic process [GO:1903607] (BP) References: PMID:19721088 Sources: GOC:TermGenie, GOC:dph, GO_REF:0000068 Also known as: cytochrome c anabolism, cytochrome c biosynthesis, cytochrome c formation, cytochrome c synthesis Relationships: is a type of GO:1903605; is_a cytochrome c metabolic process [GO:1903606] Definition: The chemical reactions and pathways resulting in the formation of cytochrome c.